{
  "gene": "UniProtKB:Q13956",
  "gene_name": "Retinal cone rhodopsin-sensitive cGMP 3',5'-cyclic phosphodiesterase subunit gamma",
  "gene_symbol": "PDE6H",
  "term_label": "positive regulation of G protein-coupled receptor signaling pathway",
  "term_id": "GO:0045745"
}